{
  "gene_symbol": "ZNF540",
  "gene_name": "Zinc finger protein 540",
  "term_id": "GO:0006357",
  "term_label": "regulation of transcription by RNA polymerase II",
  "gene": "UniProtKB:Q8NDQ6"
}